mRNA 5'-cap (guanine-N7-)-methyltransferase activity [GO:0004482] (molecular function) Relationships: is a type of N-methyltransferase activity [GO:0008170]; is a type of mRNA methyltransferase activity [GO:0008174]; is part of 7-methylguanosine mRNA capping [GO:0006370]; is part of RNA 5'-cap (guanine-N7)-methylation [GO:0106005] Also known as: S-adenosyl-L-methionine:mRNA (guanine-7-N-)-methyltransferase activity, S-adenosyl-L-methionine:mRNA (guanine-N7-)-methyltransferase activity, guanine-7-methyltransferase activity, messenger RNA guanine 7-methyltransferase activity, messenger ribonucleate guanine 7-methyltransferase activity Definition: Catalysis of the reaction: S-adenosyl-L-methionine + G(5')pppR-RNA = S-adenosyl-L-homocysteine + m7G(5')pppR-RNA. m7G(5')pppR-RNA is mRNA containing an N7-methylguanine cap; R may be guanosine or adenosine. Sources: EC:2.1.1.56